{
  "term_id": "GO:0005634",
  "gene": "UniProtKB:P10071",
  "gene_name": "Transcriptional activator GLI3",
  "gene_symbol": "GLI3",
  "term_label": "nucleus"
}